thermospermine synthase activity [GO:0010487] (MF) Relationships: is a type of transferase activity, transferring alkyl or aryl (other than methyl) groups [GO:0016765] Definition: Catalysis of the reaction: S-adenosyl-L-methioninamine + spermidine = S-methyl-5'-thioadenosine + thermospermine + H+. References: PMID:17560575 Sources: EC:2.5.1.79, MetaCyc:RXN-11190